{
  "term_id": "GO:0140807",
  "gene": "UniProtKB:Q9Y6F1",
  "gene_name": "Protein mono-ADP-ribosyltransferase PARP3",
  "gene_symbol": "PARP3",
  "term_label": "NAD+-protein-glutamate ADP-ribosyltransferase activity"
}